{
  "term_label": "DNA-binding transcription factor activity, RNA polymerase II-specific",
  "term_id": "GO:0000981",
  "gene": "UniProtKB:Q03052",
  "gene_name": "POU domain, class 3, transcription factor 1",
  "gene_symbol": "POU3F1"
}